positive regulation of mitotic division septum assembly [GO:0140281] (biological process) Definition: Any process that activates or increases the frequency, rate or extent of mitotic division septum formation. Division septum formation is the assembly and arrangement of a septum that spans the plasma membrane interface between progeny cells following cytokinesis. References: PMID:22786806 Also known as: activation of division septum formation involved in mitotic cell cycle, activation of formation of division septum involved in mitotic cell cycle, activation of mitotic division septum assembly, activation of septin assembly and septum biosynthesis involved in mitotic cell cycle, activation of septin assembly and septum formation involved in mitotic cell cycle, positive regulation of division septum formation involved in mitotic cell cycle, positive regulation of formation of division septum involved in mitotic cell cycle, positive regulation of septin assembly and septum biosynthesis involved in mitotic cell cycle, up regulation of division septum formation involved in mitotic cell cycle, up regulation of formation of division septum involved in mitotic cell cycle, up regulation of mitotic division septum assembly, up regulation of septin assembly and septum biosynthesis involved in mitotic cell cycle, up regulation of septin assembly and septum formation involved in mitotic cell cycle, up-regulation of division septum formation involved in mitotic cell cycle, up-regulation of formation of division septum involved in mitotic cell cycle, up-regulation of mitotic division septum assembly, up-regulation of septin assembly and septum biosynthesis involved in mitotic cell cycle, up-regulation of septin assembly and septum formation involved in mitotic cell cycle, upregulation of division septum formation involved in mitotic cell cycle, upregulation of formation of division septum involved in mitotic cell cycle, upregulation of septin assembly and septum biosynthesis involved in mitotic cell cycle, upregulation of septin assembly and septum formation involved in mitotic cell cycle, positive regulation of septin assembly and septum formation involved in mitotic cell cycle Relationships: is a type of positive regulation of division septum assembly [GO:0010973]; is_a regulation of mitotic division septum assembly [GO:0140279]; is a type of positive regulation of mitotic cytokinetic process [GO:1903438]; RO_0002213 GO:0140278 Subtypes: positive regulation of secondary cell septum biogenesis [GO:1903397]